{
  "term_label": "inflammatory response",
  "gene_name": "Disintegrin and metalloproteinase domain-containing protein 8",
  "term_id": "GO:0006954",
  "gene": "UniProtKB:P78325",
  "gene_symbol": "ADAM8"
}